{
  "term_id": "GO:0004984",
  "term_label": "olfactory receptor activity",
  "gene_symbol": "OR10D4P",
  "gene_name": "Putative olfactory receptor 10D4",
  "gene": "UniProtKB:Q8NGN7"
}